positive regulation of sensory perception of pain [GO:1904058] (biological process) References: PMID:17167094 Sources: GOC:TermGenie, GO_REF:0000058 Relationships: is_a positive regulation of nervous system process [GO:0031646]; is a type of regulation of sensory perception of pain [GO:0051930]; positively regulates sensory perception of pain [GO:0019233] Also known as: positive regulation of nociception, up regulation of nociception, up regulation of sensory perception of pain, up-regulation of nociception, up-regulation of sensory perception of pain, upregulation of nociception, upregulation of sensory perception of pain, activation of nociception, activation of perception of physiological pain, activation of sensory perception of pain, positive regulation of perception of physiological pain, up regulation of perception of physiological pain, up-regulation of perception of physiological pain, upregulation of perception of physiological pain Definition: Any process that activates or increases the frequency, rate or extent of sensory perception of pain.